{
  "term_id": "GO:0005739",
  "gene_name": "2,4-dienoyl-CoA reductase [(3E)-enoyl-CoA-producing], mitochondrial",
  "gene": "UniProtKB:Q16698",
  "term_label": "mitochondrion",
  "gene_symbol": "DECR1"
}